{
  "gene": "UniProtKB:Q53RE8",
  "term_label": "Unknown molecular function",
  "gene_symbol": "ANKRD39",
  "term_id": "UNKNOWN:0001",
  "gene_name": "Ankyrin repeat domain-containing protein 39"
}